{
  "term_label": "3'-UTR-mediated mRNA stabilization",
  "gene_name": "Protein boule-like",
  "term_id": "GO:0070935",
  "gene": "UniProtKB:Q8N9W6",
  "gene_symbol": "BOLL"
}